{
  "term_label": "cytosolic small ribosomal subunit",
  "term_id": "GO:0022627",
  "gene_symbol": "RPS26P11",
  "gene_name": "Putative ribosomal protein eS26-like",
  "gene": "UniProtKB:Q5JNZ5"
}